{
  "term_id": "GO:0045944",
  "gene_symbol": "BCL9L",
  "term_label": "positive regulation of transcription by RNA polymerase II",
  "gene_name": "B-cell CLL_lymphoma 9-like protein",
  "gene": "UniProtKB:Q86UU0"
}